{
  "gene": "UniProtKB:P52803",
  "gene_name": "Ephrin-A5",
  "term_id": "GO:0009897",
  "gene_symbol": "EFNA5",
  "term_label": "external side of plasma membrane"
}